{
  "term_id": "GO:0005085",
  "gene_name": "Ragulator complex protein LAMTOR5",
  "term_label": "guanyl-nucleotide exchange factor activity",
  "gene": "UniProtKB:O43504",
  "gene_symbol": "LAMTOR5"
}